pregnan-21-ol dehydrogenase (NADP+) activity [GO:0047008] (MF) Sources: RHEA:23712 Also known as: 21-hydroxy steroid (nicotinamide adenine dinucleotide phosphate) dehydrogenase activity, 21-hydroxy steroid dehydrogenase (nicotinamide adenine dinucleotide phosphate) activity, 21-hydroxy steroid dehydrogenase activity, 21-hydroxysteroid dehydrogenase (NADP+) activity, 21-hydroxysteroid:NADP+ 21-oxidoreductase activity, NADP-21-hydroxysteroid dehydrogenase activity Relationships: is a type of steroid dehydrogenase activity, acting on the CH-OH group of donors, NAD or NADP as acceptor [GO:0033764] Definition: Catalysis of the reaction: NADP+ + pregnan-21-ol = H+ + NADPH + pregnan-21-al.